{
  "gene_name": "Kelch-like protein 34",
  "gene": "UniProtKB:Q8N239",
  "term_id": "UNKNOWN:0001",
  "term_label": "Unknown molecular function",
  "gene_symbol": "KLHL34"
}